positive regulation of semaphorin-plexin signaling pathway involved in outflow tract morphogenesis [GO:2000764] (biological process) Definition: Any process that activates or increases the frequency, rate or extent of semaphorin-plexin signaling pathway involved in outflow tract morphogenesis. Sources: GOC:BHF Also known as: positive regulation of semaphorin-plexin signalling pathway involved in outflow tract morphogenesis Relationships: is a type of positive regulation of semaphorin-plexin signaling pathway [GO:2001262]; RO_0002213 GO:0071527